{
  "gene_name": "Fibroblast growth factor 4",
  "gene_symbol": "FGF4",
  "term_label": "cytoplasm",
  "gene": "UniProtKB:P08620",
  "term_id": "GO:0005737"
}